{
  "term_id": "GO:0032053",
  "gene_name": "Centriolar coiled-coil protein of 110 kDa",
  "gene": "UniProtKB:O43303",
  "gene_symbol": "CCP110",
  "term_label": "ciliary basal body organization"
}